{
  "gene": "UniProtKB:P30622",
  "term_label": "microtubule plus-end binding",
  "term_id": "GO:0051010",
  "gene_symbol": "CLIP1",
  "gene_name": "CAP-Gly domain-containing linker protein 1"
}